nitrogen utilization [GO:0019740] (biological process) Subtypes: ammonia assimilation cycle [GO:0019676] Definition: A series of processes that forms an integrated mechanism by which a cell or an organism detects the depletion of primary nitrogen source, usually ammonia, and then activates genes to scavenge the last traces of the primary nitrogen source and to transport and metabolize alternative nitrogen sources. The utilization process begins when the cell or organism detects nitrogen levels, includes the activation of genes whose products detect, transport or metabolize nitrogen-containing substances, and ends when nitrogen is incorporated into the cell or organism's metabolism. Regulation: regulated by regulation of nitrogen utilization [GO:0006808]; negatively regulated by negative regulation of nitrogen utilization [GO:0045847]; positively regulated by GO:0045848 Sources: GOC:mah, GOC:mlg Relationships: is a type of GO:0031667; is a type of intracellular nitrogen homeostasis [GO:0141067]; has part GO:0008152; has part nitrogen compound transport [GO:0071705]